{
  "gene_name": "Membrane-spanning 4-domains subfamily A member 14",
  "term_id": "UNKNOWN:0001",
  "gene": "UniProtKB:Q96JA4",
  "term_label": "Unknown molecular function",
  "gene_symbol": "MS4A14"
}